{
  "gene_name": "Homeobox protein Hox-A5",
  "gene": "UniProtKB:P20719",
  "term_label": "RNA polymerase II cis-regulatory region sequence-specific DNA binding",
  "gene_symbol": "HOXA5",
  "term_id": "GO:0000978"
}